{
  "gene": "UniProtKB:Q8N3Z6",
  "gene_symbol": "ZCCHC7",
  "gene_name": "Zinc finger CCHC domain-containing protein 7",
  "term_id": "GO:0071035",
  "term_label": "nuclear polyadenylation-dependent rRNA catabolic process"
}